negative regulation of DNA-templated DNA replication initiation [GO:0032297] (biological process) Sources: GOC:mah Relationships: is a type of regulation of DNA-templated DNA replication initiation [GO:0030174]; is a type of negative regulation of DNA-templated DNA replication [GO:2000104]; RO_0002212 DNA replication initiation [GO:0006270] Also known as: negative regulation of DNA replication initiation, down regulation of DNA replication initiation, down-regulation of DNA replication initiation, downregulation of DNA replication initiation, negative regulation of DNA-dependent DNA replication initiation, inhibition of DNA replication initiation Subtypes: negative regulation of DNA replication initiation involved in plasmid copy number maintenance [GO:0060910], negative regulation of mitotic DNA replication initiation [GO:1903467], negative regulation of initiation of premeiotic DNA replication [GO:1904513] Definition: Any process that stops, prevents, or reduces the frequency, rate or extent of initiation of DNA-dependent DNA replication.